abducens nucleus development [GO:0021742] (biological process) Sources: GOC:cls, GOC:curators, GOC:dgh, GOC:dph, GOC:jid Relationships: is a type of neural nucleus development [GO:0048857]; is part of pons development [GO:0021548] Definition: The process whose specific outcome is the progression of the abducens nucleus over time, from its formation to the mature structure.